sweet taste receptor activity [GO:0033041] (molecular function) Sources: GOC:mah Subtypes: GPCR sweet taste receptor activity [GO:0090683] Relationships: is a type of taste receptor activity [GO:0008527]; is part of detection of chemical stimulus involved in sensory perception of sweet taste [GO:0001582] Definition: Combining with soluble sweet compounds to initiate a change in cell activity. These receptors are responsible for the sense of sweet taste.